nuclear replisome [GO:0043601] (cellular component) Sources: GOC:jl, GOC:mtg_sensu Definition: A multi-component enzymatic machine at the nuclear replication fork, which mediates DNA replication. Includes DNA primase, one or more DNA polymerases, DNA helicases, and other proteins. Relationships: is a type of replisome [GO:0030894]; is a type of nuclear protein-containing complex [GO:0140513]; is part of nuclear replication fork [GO:0043596]; has part epsilon DNA polymerase complex [GO:0008622]